{
  "term_label": "nucleus",
  "gene": "UniProtKB:P84550",
  "gene_name": "SKI family transcriptional corepressor 1",
  "gene_symbol": "SKOR1",
  "term_id": "GO:0005634"
}